myosin VI complex [GO:0031476] (cellular component) Definition: A myosin complex containing one or more class VI myosin heavy chains and associated light chains. Myosin VI has a single IQ motif in the neck and a tail region with a coiled coil domain followed by a unique globular domain; a unique insertion that enables myosin VI to move towards the pointed or minus end of actin filaments. Relationships: is a type of unconventional myosin complex [GO:0016461] References: PMID:15473855